{
  "gene_name": "Leucine--tRNA ligase, cytoplasmic",
  "term_id": "GO:0006429",
  "gene_symbol": "LARS1",
  "term_label": "leucyl-tRNA aminoacylation",
  "gene": "UniProtKB:Q9P2J5"
}